{
  "gene_symbol": "CPA1",
  "gene": "UniProtKB:P15085",
  "gene_name": "Carboxypeptidase A1",
  "term_id": "GO:0006508",
  "term_label": "proteolysis"
}